pattern specification involved in pronephros development [GO:0039017] (biological process) Definition: Any developmental process that results in the creation of defined areas or spaces within the pronephros to which cells respond and eventually are instructed to differentiate. Relationships: is a type of GO:0061004; is part of GO:0048793 Also known as: pattern specification involved in pronephric kidney development Sources: GOC:mtg_kidney_jan10 Subtypes: anterior/posterior pattern specification involved in pronephros development [GO:0034672], pronephric field specification [GO:0039003], specification of pronephric tubule identity [GO:0039005], proximal/distal pattern formation involved in pronephric nephron development [GO:0072196]